{
  "term_id": "UNKNOWN:0002",
  "gene": "UniProtKB:A0A0G2JNJ9",
  "gene_name": "Uncharacterized protein",
  "term_label": "Unknown biological process",
  "gene_symbol": "A0A0G2JNJ9"
}